{
  "gene": "UniProtKB:Q06889",
  "term_id": "GO:0005634",
  "gene_symbol": "EGR3",
  "gene_name": "Early growth response protein 3",
  "term_label": "nucleus"
}